{
  "term_id": "GO:0042059",
  "gene": "UniProtKB:O43610",
  "gene_symbol": "SPRY3",
  "gene_name": "Protein sprouty homolog 3",
  "term_label": "negative regulation of epidermal growth factor receptor signaling pathway"
}